RNA polymerase III core binding [GO:0000994] (molecular function) Sources: GOC:txnOH Relationships: is a type of RNA polymerase core enzyme binding [GO:0043175] Definition: Binding to an RNA polymerase III core enzyme, a multisubunit eukaryotic nuclear RNA polymerase typically composed of seventeen subunits.